{
  "gene_name": "Uncharacterized protein C11orf96",
  "term_id": "UNKNOWN:0002",
  "gene": "UniProtKB:Q7Z7L8",
  "gene_symbol": "C11orf96",
  "term_label": "Unknown biological process"
}